{
  "term_id": "UNKNOWN:0003",
  "gene_symbol": "ZNF815P",
  "gene": "UniProtKB:A8K554",
  "gene_name": "Putative protein ZNF815",
  "term_label": "Unknown cellular component"
}